{
  "term_id": "GO:0007165",
  "gene": "UniProtKB:Q8TBJ4",
  "gene_name": "Phospholipid phosphatase-related protein type 1",
  "gene_symbol": "PLPPR1",
  "term_label": "signal transduction"
}